{
  "gene_symbol": "GGT1",
  "gene_name": "Glutathione hydrolase 1 proenzyme",
  "term_id": "GO:0002682",
  "gene": "UniProtKB:P19440",
  "term_label": "regulation of immune system process"
}